{
  "term_id": "GO:0035418",
  "gene": "UniProtKB:Q12959",
  "term_label": "protein localization to synapse",
  "gene_name": "Disks large homolog 1",
  "gene_symbol": "DLG1"
}